salicylic acid catabolic process [GO:0046244] (biological process) Relationships: is a type of salicylic acid metabolic process [GO:0009696]; is a type of GO:0019336; is a type of monocarboxylic acid catabolic process [GO:0072329] Also known as: salicylic acid breakdown, salicylic acid catabolism, salicylic acid degradation Sources: GOC:ai Definition: The chemical reactions and pathways resulting in the breakdown of salicylic acid (2-hydroxybenzoic acid), a derivative of benzoic acid.